{
  "gene": "UniProtKB:Q8IXM2",
  "gene_name": "Chromatin complexes subunit BAP18",
  "term_id": "UNKNOWN:0001",
  "gene_symbol": "BAP18",
  "term_label": "Unknown molecular function"
}